{
  "term_id": "UNKNOWN:0001",
  "gene": "UniProtKB:A8MYJ7",
  "term_label": "Unknown molecular function",
  "gene_name": "Tetratricopeptide repeat protein 34",
  "gene_symbol": "TTC34"
}